regulation of peripheral B cell anergy [GO:0002917] (biological process) Definition: Any process that modulates the frequency, rate, or extent of peripheral B cell anergy. Sources: GOC:add Relationships: is a type of regulation of peripheral tolerance induction [GO:0002658]; is a type of regulation of B cell anergy [GO:0002670]; is a type of GO:0002712; regulates GO:0002453 Subtypes: negative regulation of peripheral B cell anergy [GO:0002918], GO:0002919